{
  "term_id": "UNKNOWN:0002",
  "gene_symbol": "CCDC70",
  "term_label": "Unknown biological process",
  "gene_name": "Coiled-coil domain-containing protein 70",
  "gene": "UniProtKB:Q6NSX1"
}